{
  "term_id": "GO:0005769",
  "gene": "UniProtKB:Q15075",
  "gene_symbol": "EEA1",
  "term_label": "early endosome",
  "gene_name": "Early endosome antigen 1"
}